micturition [GO:0060073] (biological process) Sources: GOC:dph Relationships: is a type of GO:0003014; is a type of excretion [GO:0007588] Definition: The regulation of body fluids process in which parasympathetic nerves stimulate the bladder wall muscle to contract and expel urine from the body. Also known as: urination, urine voiding